{
  "gene": "UniProtKB:Q8N1V2",
  "term_id": "UNKNOWN:0002",
  "gene_symbol": "CFAP52",
  "gene_name": "Cilia- and flagella-associated protein 52",
  "term_label": "Unknown biological process"
}